small molecule catabolic process [GO:0044282] (biological process) Subtypes: hypochlorous acid catabolic process [GO:0002150], vitamin catabolic process [GO:0009111], GO:0016054, GO:0019341, urate catabolic process [GO:0019628], nucleobase-containing small molecule catabolic process [GO:0034656], GO:0042182, urea catabolic process [GO:0043419], alcohol catabolic process [GO:0046164], thiocyanate catabolic process [GO:0046265], GO:0046294, monosaccharide catabolic process [GO:0046365], ketone body catabolic process [GO:0046952] Sources: GOC:curators, GOC:vw Definition: The chemical reactions and pathways resulting in the breakdown of small molecules, any low molecular weight, monomeric, non-encoded molecule. Relationships: is a type of catabolic process [GO:0009056]; is a type of GO:0044281 Also known as: small molecule catabolism Note: Small molecules in GO include monosaccharides but exclude disaccharides and polysaccharides.